negative regulation of guanyl-nucleotide exchange factor activity [GO:1905098] (biological process) Definition: Any process that stops, prevents or reduces the frequency, rate or extent of guanyl-nucleotide exchange factor activity. Relationships: is a type of GO:0043087; is a type of negative regulation of molecular function [GO:0044092]; is a type of positive regulation of binding [GO:0051099]; negatively regulates GO:0005085 Subtypes: GO:2001107 Also known as: down regulation of GDP-dissociation stimulator activity, down regulation of GDS, down regulation of GEF, down regulation of guanyl-nucleotide exchange factor activity, down regulation of guanyl-nucleotide release factor activity, down regulation of guanyl-nucleotide releasing factor, down-regulation of GDP-dissociation stimulator activity, down-regulation of GDS, down-regulation of GEF, down-regulation of guanyl-nucleotide exchange factor activity, down-regulation of guanyl-nucleotide release factor activity, down-regulation of guanyl-nucleotide releasing factor, downregulation of GDP-dissociation stimulator activity, downregulation of GDS, downregulation of GEF, downregulation of guanyl-nucleotide exchange factor activity, downregulation of guanyl-nucleotide release factor activity, downregulation of guanyl-nucleotide releasing factor, negative regulation of GDP-dissociation stimulator activity, negative regulation of GDS, negative regulation of GEF, negative regulation of guanyl-nucleotide release factor activity, negative regulation of guanyl-nucleotide releasing factor, down regulation of GNRP, down-regulation of GNRP, downregulation of GNRP, inhibition of GDP-dissociation stimulator activity, inhibition of GDS, inhibition of GEF, inhibition of GNRP, inhibition of guanyl-nucleotide exchange factor activity, inhibition of guanyl-nucleotide release factor activity, inhibition of guanyl-nucleotide releasing factor, negative regulation of GNRP References: PMID:20484009 Sources: GOC:TermGenie, GO_REF:0000059